CENP-A eviction from euchromatin [GO:0140898] (biological process) Relationships: is a type of chromatin remodeling [GO:0006338] Definition: A chromatin remodeling process in which CENP-A is removed from euchromatin regions to prevent neocentromere formation. References: PMID:27666591